{
  "term_label": "actin filament polymerization",
  "gene_symbol": "DIAPH3",
  "gene_name": "Protein diaphanous homolog 3",
  "gene": "UniProtKB:Q9NSV4",
  "term_id": "GO:0030041"
}